{
  "term_label": "Unknown biological process",
  "gene_symbol": "CCDC78",
  "gene": "UniProtKB:A2IDD5",
  "term_id": "UNKNOWN:0002",
  "gene_name": "Coiled-coil domain-containing protein 78"
}